{
  "gene_name": "Myelin-associated oligodendrocyte basic protein",
  "gene_symbol": "MOBP",
  "term_id": "UNKNOWN:0003",
  "gene": "UniProtKB:Q13875",
  "term_label": "Unknown cellular component"
}